{
  "gene_symbol": "LIN7A",
  "gene_name": "Protein lin-7 homolog A",
  "gene": "UniProtKB:O14910",
  "term_label": "synapse",
  "term_id": "GO:0045202"
}